{
  "gene_symbol": "IGHJ4",
  "term_label": "Unknown molecular function",
  "term_id": "UNKNOWN:0001",
  "gene_name": "Immunoglobulin heavy joining 4 (Fragment)",
  "gene": "UniProtKB:A0A0J9YVS3"
}